{
  "gene_symbol": "LPAR6",
  "gene_name": "Lysophosphatidic acid receptor 6",
  "term_id": "GO:0007186",
  "gene": "UniProtKB:P43657",
  "term_label": "G protein-coupled receptor signaling pathway"
}